plasma membrane signaling receptor complex [GO:0098802] (cellular component) Subtypes: GO:0005892, GO:0005893, interleukin-3 receptor complex [GO:0005894], interleukin-5 receptor complex [GO:0005895], GO:0005896, GO:0005897, interleukin-13 receptor complex [GO:0005898], insulin receptor complex [GO:0005899], GO:0005900, integrin complex [GO:0008305], GO:0016516, GO:0019815, GO:0030526, interleukin-20 receptor complex [GO:0030876], high molecular weight kininogen receptor complex [GO:0030988], interleukin-28 receptor complex [GO:0032002], Toll-like receptor 1-Toll-like receptor 2 protein complex [GO:0035354], GO:0035355, CD40 receptor complex [GO:0035631], ERBB4-EGFR complex [GO:0038139], ERBB4-ERBB3 complex [GO:0038140], GO:0038141, EGFR:ERBB2 complex [GO:0038142], ERBB3:ERBB2 complex [GO:0038143], ERBB4:ERBB2 complex [GO:0038144], type I interferon receptor complex [GO:0038197], GO:0042022, GO:0042101, pre-T cell receptor complex [GO:0043384], interleukin-18 receptor complex [GO:0045092], interleukin-1 receptor complex [GO:0045323], activin receptor complex [GO:0048179], transforming growth factor beta ligand-receptor complex [GO:0070021], ciliary neurotrophic factor receptor complex [GO:0070110], BMP receptor complex [GO:0070724], interleukin-23 receptor complex [GO:0072536], G protein-coupled receptor complex [GO:0097648], neurotransmitter receptor complex [GO:0098878], HFE-transferrin receptor complex [GO:1990712], glycoprotein Ib-IX-V complex [GO:1990779], humanin receptor complex [GO:7770013] Note: Note that this term is in the subset of terms that should not be used for direct gene product annotation. Instead, select a child term or, if no appropriate child term exists, please request a new term. Direct annotations to this term may be amended during annotation QC. Definition: Any protein complex that is part of the plasma membrane and which functions as a signaling receptor. Sources: GOC:dos Relationships: is a type of GO:0043235; is a type of plasma membrane protein complex [GO:0098797]